{
  "term_id": "GO:0016020",
  "term_label": "membrane",
  "gene_symbol": "OR10K2",
  "gene_name": "Olfactory receptor 10K2",
  "gene": "UniProtKB:Q6IF99"
}